{
  "term_id": "GO:2000042",
  "gene": "UniProtKB:Q8IYI0",
  "gene_symbol": "SHLD1",
  "term_label": "negative regulation of double-strand break repair via homologous recombination",
  "gene_name": "Shieldin complex subunit 1"
}